{
  "term_id": "GO:0004984",
  "gene_symbol": "OR51B2",
  "gene_name": "Olfactory receptor 51B2",
  "term_label": "olfactory receptor activity",
  "gene": "UniProtKB:Q9Y5P1"
}